{
  "term_id": "GO:0008210",
  "gene_name": "UDP-glucuronosyltransferase 2B17",
  "gene_symbol": "UGT2B17",
  "gene": "UniProtKB:O75795",
  "term_label": "estrogen metabolic process"
}